high-affinity phosphate:sodium symporter activity [GO:0005316] (MF) Sources: TC:2.A.20.2.2 Definition: Enables the transfer of a solute or solutes from one side of a membrane to the other according to the reaction:phosphate(out) + Na+(out) = phosphate(in) + Na+(in). In high-affinity transport the transporter is able to bind the solute even if it is only present at very low concentrations. Relationships: is a type of GO:0005436 Also known as: sodium/phosphate cotransporter activity, high affinity inorganic phosphate:sodium symporter activity, high-affinity inorganic phosphate:sodium symporter activity